{
  "term_label": "3-hydroxyacyl-CoA dehydratase activity",
  "term_id": "GO:0018812",
  "gene_name": "Very-long-chain (3R)-3-hydroxyacyl-CoA dehydratase 4",
  "gene_symbol": "HACD4",
  "gene": "UniProtKB:Q5VWC8"
}